{
  "term_label": "protein import into nucleus",
  "gene_name": "Nuclear pore glycoprotein p62",
  "gene_symbol": "NUP62",
  "term_id": "GO:0006606",
  "gene": "UniProtKB:P37198"
}